{
  "gene_symbol": "C9orf43",
  "gene": "UniProtKB:Q8TAL5",
  "gene_name": "Uncharacterized protein C9orf43",
  "term_label": "Unknown molecular function",
  "term_id": "UNKNOWN:0001"
}